{
  "gene_symbol": "UMPS",
  "gene": "UniProtKB:P11172",
  "term_id": "UNKNOWN:0003",
  "term_label": "Unknown cellular component",
  "gene_name": "Uridine 5'-monophosphate synthase"
}